{
  "gene": "UniProtKB:E5RJ46",
  "term_label": "Unknown cellular component",
  "gene_symbol": "LINC02906",
  "gene_name": "Putative uncharacterized protein LINC02906",
  "term_id": "UNKNOWN:0003"
}